regulation of hindgut contraction [GO:0043134] (biological process) Definition: Any process that modulates the frequency, rate or extent of muscle contraction of the hindgut, the posterior part of the alimentary canal, including the rectum, and the large intestine. Sources: GOC:jl, UBERON:0001046 Subtypes: positive regulation of hindgut contraction [GO:0060450], negative regulation of hindgut contraction [GO:0060451] Relationships: is a type of GO:0006940; is a type of regulation of digestive system process [GO:0044058]; regulates hindgut contraction [GO:0043133]